{
  "gene_symbol": "FGF17",
  "term_label": "extracellular space",
  "gene": "UniProtKB:O60258",
  "term_id": "GO:0005615",
  "gene_name": "Fibroblast growth factor 17"
}